{
  "term_id": "GO:0030688",
  "term_label": "preribosome, small subunit precursor",
  "gene": "UniProtKB:Q13895",
  "gene_name": "Bystin",
  "gene_symbol": "BYSL"
}